{
  "term_id": "GO:0033038",
  "term_label": "bitter taste receptor activity",
  "gene_symbol": "TAS2R13",
  "gene": "UniProtKB:Q9NYV9",
  "gene_name": "Taste receptor type 2 member 13"
}